{
  "term_label": "proteasome-mediated ubiquitin-dependent protein catabolic process",
  "term_id": "GO:0043161",
  "gene": "UniProtKB:Q8NFY9",
  "gene_symbol": "KBTBD8",
  "gene_name": "Kelch repeat and BTB domain-containing protein 8"
}